{
  "term_label": "intermediate filament organization",
  "gene_name": "Keratin, type I cytoskeletal 25",
  "gene": "UniProtKB:Q7Z3Z0",
  "gene_symbol": "KRT25",
  "term_id": "GO:0045109"
}